{
  "gene_symbol": "MEP1B",
  "gene_name": "Meprin A subunit beta",
  "term_label": "Unknown biological process",
  "gene": "UniProtKB:Q16820",
  "term_id": "UNKNOWN:0002"
}